{
  "gene": "UniProtKB:Q9BS26",
  "term_id": "GO:0003756",
  "gene_name": "Endoplasmic reticulum resident protein 44",
  "term_label": "protein disulfide isomerase activity",
  "gene_symbol": "ERP44"
}